{
  "gene": "UniProtKB:Q92564",
  "term_label": "cullin family protein binding",
  "gene_name": "DCN1-like protein 4",
  "gene_symbol": "DCUN1D4",
  "term_id": "GO:0097602"
}